{
  "gene_symbol": "PAQR3",
  "gene": "UniProtKB:Q6TCH7",
  "term_id": "GO:0005794",
  "gene_name": "Progestin and adipoQ receptor family member 3",
  "term_label": "Golgi apparatus"
}